{
  "term_id": "GO:0005829",
  "term_label": "cytosol",
  "gene": "UniProtKB:O75688",
  "gene_name": "Protein phosphatase 1B",
  "gene_symbol": "PPM1B"
}